{
  "gene": "UniProtKB:Q4G163",
  "gene_name": "F-box only protein 43",
  "gene_symbol": "FBXO43",
  "term_id": "UNKNOWN:0001",
  "term_label": "Unknown molecular function"
}